{
  "term_id": "GO:0005829",
  "gene_name": "Trafficking protein particle complex subunit 3-like protein",
  "term_label": "cytosol",
  "gene_symbol": "TRAPPC3L",
  "gene": "UniProtKB:Q5T215"
}